{
  "gene_name": "S1 RNA-binding domain-containing protein 1",
  "term_label": "mRNA binding",
  "gene_symbol": "SRBD1",
  "term_id": "GO:0003729",
  "gene": "UniProtKB:Q8N5C6"
}